{
  "term_label": "synapse maturation",
  "gene_name": "Paralemmin-1",
  "term_id": "GO:0060074",
  "gene": "UniProtKB:O75781",
  "gene_symbol": "PALM"
}